{
  "term_id": "GO:0031573",
  "term_label": "mitotic intra-S DNA damage checkpoint signaling",
  "gene_name": "Probable crossover junction endonuclease EME2",
  "gene": "UniProtKB:A4GXA9",
  "gene_symbol": "EME2"
}